{
  "gene": "UniProtKB:P60411",
  "gene_name": "Keratin-associated protein 10-9",
  "term_label": "Unknown molecular function",
  "gene_symbol": "KRTAP10-9",
  "term_id": "UNKNOWN:0001"
}